{
  "gene": "UniProtKB:Q8NEP9",
  "gene_symbol": "ZNF555",
  "gene_name": "Zinc finger protein 555",
  "term_label": "RNA polymerase II transcription regulatory region sequence-specific DNA binding",
  "term_id": "GO:0000977"
}